{
  "term_id": "GO:0003682",
  "gene_symbol": "SAMD7",
  "term_label": "chromatin binding",
  "gene_name": "Sterile alpha motif domain-containing protein 7",
  "gene": "UniProtKB:Q7Z3H4"
}